{
  "gene": "UniProtKB:P32927",
  "term_label": "interleukin-3-mediated signaling pathway",
  "term_id": "GO:0038156",
  "gene_name": "Cytokine receptor common subunit beta",
  "gene_symbol": "CSF2RB"
}